{
  "gene": "UniProtKB:Q9C0J9",
  "gene_name": "Class E basic helix-loop-helix protein 41",
  "gene_symbol": "BHLHE41",
  "term_label": "nucleus",
  "term_id": "GO:0005634"
}